{
  "term_label": "regulation of Rab protein signal transduction",
  "gene": "UniProtKB:Q8WXG6",
  "term_id": "GO:0032483",
  "gene_symbol": "MADD",
  "gene_name": "MAP kinase-activating death domain protein"
}